{
  "term_label": "cytoplasm",
  "gene": "UniProtKB:P50461",
  "gene_name": "Cysteine and glycine-rich protein 3",
  "gene_symbol": "CSRP3",
  "term_id": "GO:0005737"
}